branching involved in prostate gland morphogenesis [GO:0060442] (biological process) Regulation: regulated by regulation of branching involved in prostate gland morphogenesis [GO:0060687] Sources: GOC:dph Definition: The process in which the branching structure of the prostate gland is generated and organized. A branch is a division or offshoot from a main stem. Relationships: is a type of GO:0060740; is a type of morphogenesis of a branching epithelium [GO:0061138] Also known as: prostate gland branching morphogenesis, prostate branching Subtypes: GO:0060527